{
  "gene_symbol": "CCDC69",
  "gene_name": "Coiled-coil domain-containing protein 69",
  "term_label": "nucleus",
  "term_id": "GO:0005634",
  "gene": "UniProtKB:A6NI79"
}